{
  "gene": "UniProtKB:P14653",
  "term_id": "GO:0005634",
  "gene_symbol": "HOXB1",
  "gene_name": "Homeobox protein Hox-B1",
  "term_label": "nucleus"
}